{
  "term_id": "GO:0030036",
  "gene": "UniProtKB:Q9Y4G6",
  "term_label": "actin cytoskeleton organization",
  "gene_symbol": "TLN2",
  "gene_name": "Talin-2"
}